nitrate transmembrane transport [GO:0015706] (biological process) Definition: The directed movement of nitrate into, out of or within a cell, or between cells, by means of some agent such as a transporter or pore. Sources: GOC:krc Also known as: nitrate transport, low affinity nitrate transport, low-affinity nitrate transport Relationships: is a type of transmembrane transport [GO:0055085]; is a type of nitrate import [GO:1902025] Subtypes: phloem nitrate loading [GO:0090408]